Gram-negative-bacterium-type cell wall [GO:0009276] (cellular component) Definition: The peptidoglycan layer of the Gram-negative cell envelope. In Gram-negative cells the peptidoglycan is relatively thin (1-2nm) and is linked to the outer membrane by lipoproteins. In Gram-negative cells the peptidoglycan is too thin to retain the primary stain in the Gram staining procedure and therefore cells appear red after Gram stain. Sources: GOC:mlg, ISBN:0815108893 Also known as: 1-2nm peptidoglycan-based cell wall, cell wall inner membrane Relationships: is_a peptidoglycan-based cell wall [GO:0009274]; is part of cell envelope [GO:0030313]